{
  "gene": "UniProtKB:P55773",
  "term_label": "positive regulation of cell migration",
  "gene_name": "C-C motif chemokine 23",
  "gene_symbol": "CCL23",
  "term_id": "GO:0030335"
}